{
  "gene_symbol": "F9",
  "term_id": "GO:0004252",
  "term_label": "serine-type endopeptidase activity",
  "gene": "UniProtKB:P00740",
  "gene_name": "Coagulation factor IX"
}